{
  "gene": "UniProtKB:Q5SQS8",
  "term_id": "UNKNOWN:0001",
  "term_label": "Unknown molecular function",
  "gene_symbol": "C10orf120",
  "gene_name": "Uncharacterized protein C10orf120"
}